calcium ion import [GO:0070509] (biological process) Regulation: regulated by regulation of calcium ion import [GO:0090279]; positively regulated by positive regulation of calcium ion import [GO:0090280]; negatively regulated by negative regulation of calcium ion import [GO:0090281] Sources: GOC:mah Also known as: calcium ion uptake, transmembrane calcium influx Subtypes: calcium ion import across plasma membrane [GO:0098703] Definition: The directed movement of calcium ions into a cell or organelle. Relationships: is a type of calcium ion transport [GO:0006816]